{
  "term_id": "UNKNOWN:0002",
  "gene_symbol": "MUC16",
  "gene_name": "Mucin-16",
  "gene": "UniProtKB:Q8WXI7",
  "term_label": "Unknown biological process"
}